{
  "term_label": "NADP binding",
  "gene_symbol": "DPYD",
  "gene_name": "Dihydropyrimidine dehydrogenase [NADP(+)]",
  "gene": "UniProtKB:Q12882",
  "term_id": "GO:0050661"
}